adhesion of symbiont haustorium mother cell to host [GO:0075196] (biological process) Relationships: is a type of adhesion of symbiont infection structure to host [GO:0075001] Sources: GOC:pamgo_curators Definition: The attachment of a haustorium mother cell of the symbiont to its host via adhesion molecules. The host is defined as the larger of the organisms involved in a symbiotic interaction. Also known as: adhesion of symbiont haustorium mother cell to host during symbiotic interaction Note: Note that this term should not be used to annotate gene products of the host. It should only be used to annotate those gene products from the symbiont involved in this process.